{
  "gene": "UniProtKB:Q9BQJ4",
  "gene_symbol": "TMEM47",
  "gene_name": "Transmembrane protein 47",
  "term_label": "cell-cell junction",
  "term_id": "GO:0005911"
}